{
  "gene": "UniProtKB:Q9BQG1",
  "gene_symbol": "SYT3",
  "term_label": "calcium ion sensor activity",
  "term_id": "GO:0061891",
  "gene_name": "Synaptotagmin-3"
}